{
  "gene": "UniProtKB:P58215",
  "gene_name": "Lysyl oxidase homolog 3",
  "term_id": "GO:0031012",
  "term_label": "extracellular matrix",
  "gene_symbol": "LOXL3"
}